{
  "term_id": "GO:0005634",
  "term_label": "nucleus",
  "gene_name": "Adenylate kinase isoenzyme 6",
  "gene": "UniProtKB:Q9Y3D8",
  "gene_symbol": "AK6"
}